{
  "term_label": "intermediate filament",
  "gene": "UniProtKB:P48681",
  "term_id": "GO:0005882",
  "gene_symbol": "NES",
  "gene_name": "Nestin"
}